{
  "gene_symbol": "CXCL9",
  "term_label": "CXCR chemokine receptor binding",
  "gene_name": "C-X-C motif chemokine 9",
  "gene": "UniProtKB:Q07325",
  "term_id": "GO:0045236"
}